{
  "gene_symbol": "CFAP410",
  "term_label": "Unknown molecular function",
  "gene_name": "Cilia- and flagella-associated protein 410",
  "gene": "UniProtKB:O43822",
  "term_id": "UNKNOWN:0001"
}